{
  "term_label": "nuclear export",
  "term_id": "GO:0051168",
  "gene": "UniProtKB:P49792",
  "gene_name": "E3 SUMO-protein ligase RanBP2",
  "gene_symbol": "RANBP2"
}